{
  "gene": "UniProtKB:Q15013",
  "gene_symbol": "MAD2L1BP",
  "term_label": "Unknown molecular function",
  "term_id": "UNKNOWN:0001",
  "gene_name": "MAD2L1-binding protein"
}